{
  "gene": "UniProtKB:Q9P2W7",
  "term_id": "GO:0000139",
  "gene_name": "Galactosylgalactosylxylosylprotein 3-beta-glucuronosyltransferase 1",
  "gene_symbol": "B3GAT1",
  "term_label": "Golgi membrane"
}